{
  "term_label": "integrator complex",
  "gene_name": "Integrator complex subunit 15",
  "gene": "UniProtKB:Q96N11",
  "gene_symbol": "INTS15",
  "term_id": "GO:0032039"
}